1,5-anhydro-D-fructose dehydratase activity [GO:0033992] (molecular function) Sources: EC:4.2.1.111 Relationships: is a type of GO:0016836 Definition: Catalysis of the reaction: 1,5-anhydro-D-fructose = 1,5-anhydro-4-deoxy-D-glycero-hex-3-en-2-ulose + H2O. Also known as: 1,5-anhydro-D-arabino-hex-2-ulose dehydratase activity, 1,5-anhydro-D-fructose 4-dehydratase activity, 1,5-anhydro-D-fructose hydro-lyase (ascopyrone-M-forming) activity, 1,5-anhydro-D-fructose hydro-lyase activity, 1,5-anhydro-D-fructose hydrolyase activity, AF dehydratase activity, AFDH